{
  "term_id": "GO:0005737",
  "gene_symbol": "WARS1",
  "gene_name": "Tryptophan--tRNA ligase, cytoplasmic",
  "gene": "UniProtKB:P23381",
  "term_label": "cytoplasm"
}